{
  "gene_name": "Protein FRG2-like-1",
  "gene": "UniProtKB:Q96QU4",
  "term_label": "Unknown biological process",
  "gene_symbol": "FRG2B",
  "term_id": "UNKNOWN:0002"
}